{
  "gene_name": "Glial cell line-derived neurotrophic factor",
  "gene": "UniProtKB:P39905",
  "term_label": "growth factor activity",
  "gene_symbol": "GDNF",
  "term_id": "GO:0008083"
}